{
  "gene": "UniProtKB:Q99733",
  "term_id": "GO:0000785",
  "gene_name": "Nucleosome assembly protein 1-like 4",
  "gene_symbol": "NAP1L4",
  "term_label": "chromatin"
}